{
  "term_id": "GO:0006355",
  "term_label": "regulation of DNA-templated transcription",
  "gene_name": "Tesmin",
  "gene": "UniProtKB:Q9Y4I5",
  "gene_symbol": "TESMIN"
}